{
  "term_id": "GO:0000981",
  "term_label": "DNA-binding transcription factor activity, RNA polymerase II-specific",
  "gene_name": "Zinc finger protein 737",
  "gene_symbol": "ZNF737",
  "gene": "UniProtKB:O75373"
}